{
  "term_label": "lamellipodium",
  "gene": "UniProtKB:Q92558",
  "gene_symbol": "WASF1",
  "term_id": "GO:0030027",
  "gene_name": "Actin-binding protein WASF1"
}